{
  "gene_symbol": "MRPL1",
  "gene_name": "Large ribosomal subunit protein uL1m",
  "term_id": "GO:0006417",
  "term_label": "regulation of translation",
  "gene": "UniProtKB:Q9BYD6"
}